{
  "term_label": "Unknown biological process",
  "gene_name": "Post-GPI attachment to proteins factor 6",
  "gene_symbol": "PGAP6",
  "gene": "UniProtKB:Q9HCN3",
  "term_id": "UNKNOWN:0002"
}